pathogen-associated molecular pattern receptor signaling pathway [GO:0140426] (biological process) Relationships: is a type of GO:0002221 References: PMID:25744358 Also known as: MAMP-triggered immunity signalling, PAMP receptor signaling pathway, PAMP-triggered immunity signalling pathway, PTI signalling, pathogen-associated molecular pattern signalling Definition: The series of molecular signals initiated by a ligand binding of a pattern recognition receptor (PRR) to activate a plant innate immune response. PAMP-triggered immunity PRRs bind pathogen-associated molecular pattern (PAMPs), structures conserved among microbial species.